{
  "gene": "UniProtKB:O94888",
  "gene_symbol": "UBXN7",
  "term_id": "GO:0043161",
  "gene_name": "UBX domain-containing protein 7",
  "term_label": "proteasome-mediated ubiquitin-dependent protein catabolic process"
}